{
  "gene_symbol": "NHERF1",
  "gene": "UniProtKB:O14745",
  "term_label": "protein localization to plasma membrane",
  "gene_name": "Na(+)_H(+) exchange regulatory cofactor NHE-RF1",
  "term_id": "GO:0072659"
}